interleukin-19-mediated signaling pathway [GO:0140854] (biological process) Relationships: is a type of cytokine-mediated signaling pathway [GO:0019221] References: PMID:34052656 Definition: The series of molecular signals initiated by interleukin-19 binding to its receptor on the surface of a target cell, and ending with the regulation of a downstream cellular process, e.g. transcription. Also known as: IL19-mediated signalling pathway